{
  "gene_name": "Cyclin-dependent kinase 12",
  "term_label": "nucleus",
  "gene": "UniProtKB:Q9NYV4",
  "term_id": "GO:0005634",
  "gene_symbol": "CDK12"
}